{
  "gene_symbol": "ATG14",
  "gene": "UniProtKB:Q6ZNE5",
  "gene_name": "Beclin 1-associated autophagy-related key regulator",
  "term_id": "GO:0005776",
  "term_label": "autophagosome"
}